{
  "gene": "UniProtKB:Q05516",
  "term_id": "GO:0000978",
  "gene_name": "Zinc finger and BTB domain-containing protein 16",
  "gene_symbol": "ZBTB16",
  "term_label": "RNA polymerase II cis-regulatory region sequence-specific DNA binding"
}